neutral amino acid transmembrane export from vacuole [GO:0034489] (biological process) Subtypes: L-cystine transmembrane transport from lysosomal lumen to cytosol [GO:1904919] Sources: GOC:mah Definition: The directed movement of neutral amino acids out of the vacuole, across the vacuolar membrane. Relationships: is a type of neutral amino acid transport [GO:0015804]; is_a amino acid transmembrane export from vacuole [GO:0032974]